{
  "gene": "UniProtKB:Q96E35",
  "gene_symbol": "ZMYND19",
  "term_label": "membrane",
  "term_id": "GO:0016020",
  "gene_name": "Zinc finger MYND domain-containing protein 19"
}